BRE binding [GO:0042835] (molecular function) References: PMID:10893231 Definition: Binding to a BRE RNA element (Bruno response element). Relationships: is a type of GO:0003723